{
  "term_label": "nucleus",
  "gene_symbol": "LMCD1",
  "term_id": "GO:0005634",
  "gene_name": "LIM and cysteine-rich domains protein 1",
  "gene": "UniProtKB:Q9NZU5"
}